regulation of cell growth [GO:0001558] (biological process) Definition: Any process that modulates the frequency, rate, extent or direction of cell growth. Sources: GOC:go_curators Relationships: is a type of regulation of growth [GO:0040008]; is a type of regulation of cellular component organization [GO:0051128]; regulates GO:0016049 Subtypes: regulation of cell growth by extracellular stimulus [GO:0001560], positive regulation of cell growth [GO:0030307], negative regulation of cell growth [GO:0030308], regulation of unidimensional cell growth [GO:0051510], GO:0061050, regulation of extent of cell growth [GO:0061387], regulation of rate of cell growth [GO:0061388], GO:0061389, GO:1902890, regulation of chondrocyte hypertrophy [GO:1903041], regulation of dendrite extension [GO:1903859], regulation of pseudohyphal growth [GO:2000220]